{
  "term_id": "GO:0043161",
  "gene": "UniProtKB:Q9H871",
  "gene_name": "E3 ubiquitin-protein transferase RMND5A",
  "gene_symbol": "RMND5A",
  "term_label": "proteasome-mediated ubiquitin-dependent protein catabolic process"
}